negative regulation of membrane repolarization during cardiac muscle cell action potential [GO:1905032] (biological process) Subtypes: GO:1905001, GO:1905025 Relationships: is a type of GO:0048519; is a type of regulation of membrane repolarization during cardiac muscle cell action potential [GO:1905031]; negatively regulates membrane repolarization during cardiac muscle cell action potential [GO:0086013] Definition: Any process that stops, prevents or reduces the frequency, rate or extent of membrane repolarization during cardiac muscle cell action potential. Also known as: down regulation of membrane repolarization during cardiac muscle cell action potential, down-regulation of membrane repolarization during cardiac muscle cell action potential, downregulation of membrane repolarization during cardiac muscle cell action potential, inhibition of membrane repolarization during cardiac muscle cell action potential References: PMID:23157812 Sources: GOC:BHF, GOC:BHF_miRNA, GOC:TermGenie, GOC:mtg_cardiac_conduct_nov11, GOC:rph